{
  "gene_name": "Zinc finger protein 107",
  "gene_symbol": "ZNF107",
  "term_label": "transcription cis-regulatory region binding",
  "term_id": "GO:0000976",
  "gene": "UniProtKB:Q9UII5"
}